{
  "gene_symbol": "ATAD3B",
  "gene": "UniProtKB:Q5T9A4",
  "term_label": "Unknown molecular function",
  "gene_name": "ATPase family AAA domain-containing protein 3B",
  "term_id": "UNKNOWN:0001"
}